{
  "term_label": "synaptic vesicle membrane",
  "term_id": "GO:0030672",
  "gene_name": "Synaptotagmin-8",
  "gene_symbol": "SYT8",
  "gene": "UniProtKB:Q8NBV8"
}